{
  "gene_name": "Meteorin-like protein",
  "gene_symbol": "METRNL",
  "term_label": "extracellular space",
  "term_id": "GO:0005615",
  "gene": "UniProtKB:Q641Q3"
}